{
  "gene_name": "Motile sperm domain-containing protein 1",
  "term_label": "Unknown biological process",
  "gene": "UniProtKB:Q9UJG1",
  "gene_symbol": "MOSPD1",
  "term_id": "UNKNOWN:0002"
}